spine apparatus lumen [GO:0098899] (cellular component) Relationships: is_a cytoplasmic vesicle lumen [GO:0060205]; is part of GO:0097444 Definition: The volume enclosed by the spine apparatus membrane. Sources: GOC:dos